{
  "gene_symbol": "KRT15",
  "gene_name": "Keratin, type I cytoskeletal 15",
  "term_label": "keratin filament",
  "term_id": "GO:0045095",
  "gene": "UniProtKB:P19012"
}